{
  "gene": "UniProtKB:Q06547",
  "term_label": "transcription cis-regulatory region binding",
  "term_id": "GO:0000976",
  "gene_name": "GA-binding protein subunit beta-1",
  "gene_symbol": "GABPB1"
}